{
  "gene_symbol": "S100P",
  "gene_name": "Protein S100-P",
  "gene": "UniProtKB:P25815",
  "term_label": "calcium ion binding",
  "term_id": "GO:0005509"
}